{
  "gene_symbol": "NTM-AS1",
  "gene_name": "Putative uncharacterized protein NTM-AS1",
  "gene": "UniProtKB:Q6ZSK4",
  "term_id": "UNKNOWN:0001",
  "term_label": "Unknown molecular function"
}